{
  "term_label": "actin filament binding",
  "gene": "UniProtKB:Q14331",
  "gene_symbol": "FRG1",
  "term_id": "GO:0051015",
  "gene_name": "Protein FRG1"
}